{
  "gene_symbol": "NEK5",
  "gene_name": "Serine_threonine-protein kinase Nek5",
  "term_label": "Unknown biological process",
  "gene": "UniProtKB:Q6P3R8",
  "term_id": "UNKNOWN:0002"
}